{
  "gene_name": "Malignant T-cell-amplified sequence 2",
  "term_label": "formation of translation preinitiation complex",
  "gene_symbol": "MCTS2",
  "gene": "UniProtKB:A0A3B3IRV3",
  "term_id": "GO:0001731"
}